{
  "term_id": "UNKNOWN:0001",
  "term_label": "Unknown molecular function",
  "gene": "UniProtKB:Q2TAC2",
  "gene_name": "Coiled-coil domain-containing protein 57",
  "gene_symbol": "CCDC57"
}